{
  "gene": "UniProtKB:Q08495",
  "gene_symbol": "DMTN",
  "term_id": "GO:0030032",
  "term_label": "lamellipodium assembly",
  "gene_name": "Dematin"
}